{
  "gene": "UniProtKB:Q9HAU8",
  "gene_name": "Aminopeptidase RNPEPL1",
  "gene_symbol": "RNPEPL1",
  "term_label": "metalloaminopeptidase activity",
  "term_id": "GO:0070006"
}